{
  "gene_name": "BCL2_adenovirus E1B 19 kDa protein-interacting protein 3-like",
  "term_label": "Unknown molecular function",
  "gene": "UniProtKB:O60238",
  "term_id": "UNKNOWN:0001",
  "gene_symbol": "BNIP3L"
}